interleukin-24 production [GO:0032628] (biological process) Relationships: is a type of cytokine production [GO:0001816] Regulation: regulated by regulation of interleukin-24 production [GO:0032668]; negatively regulated by negative regulation of interleukin-24 production [GO:0032708]; positively regulated by positive regulation of interleukin-24 production [GO:0032748] Sources: GOC:mah Definition: The appearance of interleukin-24 due to biosynthesis or secretion following a cellular stimulus, resulting in an increase in its intracellular or extracellular levels. Also known as: IL-24 production, MDA7 production, ST16 production, interleukin-24 biosynthetic process, interleukin-24 secretion